{
  "gene_symbol": "ARR3",
  "term_label": "G protein-coupled receptor internalization",
  "gene_name": "Arrestin-C",
  "term_id": "GO:0002031",
  "gene": "UniProtKB:P36575"
}